N-acetylglucosaminylphosphatidylinositol deacetylase activity [GO:0000225] (molecular function) Relationships: is a type of hydrolase activity, acting on carbon-nitrogen (but not peptide) bonds, in linear amides [GO:0016811]; is a type of deacetylase activity [GO:0019213] Sources: EC:3.5.1.89 Definition: Catalysis of the reaction: N-acetyl-D-glucosaminylphosphatidylinositol + H2O = D-glucosaminylphosphatidylinositol + acetate. This reaction is the second step of the biosynthesis of glycosylphosphatidylinositol (GPI), used to anchor various eukaryotic proteins to the cell-surface membrane. Also known as: 6-(N-acetyl-alpha-D-glucosaminyl)-1-phosphatidyl-1D-myo-inositol acetylhydrolase activity, GlcNAc-PI de-N-acetylase activity, GlcNAc-PI deacetylase activity, N-acetyl-D-glucosaminylphosphatidylinositol acetylhydrolase activity, N-acetylglucosaminylphosphatidylinositol de-N-acetylase activity, acetylglucosaminylphosphatidylinositol deacetylase activity